peptidoglycan-associated peptide transport [GO:0015834] (biological process) Relationships: is a type of peptide transport [GO:0015833] Also known as: murein peptide transport, muropeptide transport, peptidoglycan peptide transport Sources: ISBN:0198506732 Definition: The directed movement of peptidoglycan peptides into, out of or within a cell, or between cells, by means of some agent such as a transporter or pore. Peptidoglycan peptides are the oligopeptides found in peptidoglycan networks which cross-link the polysaccharide chains.